{
  "term_label": "Unknown molecular function",
  "term_id": "UNKNOWN:0001",
  "gene_name": "Melanocyte protein PMEL",
  "gene": "UniProtKB:P40967",
  "gene_symbol": "PMEL"
}